{
  "term_label": "inner dynein arm",
  "gene": "UniProtKB:Q8WXX0",
  "gene_symbol": "DNAH7",
  "term_id": "GO:0036156",
  "gene_name": "Dynein axonemal heavy chain 7"
}